macrophage colony-stimulating factor receptor binding [GO:0005157] (molecular function) Definition: Binding to a macrophage colony-stimulating factor receptor. Sources: GOC:ai Also known as: M-CSF receptor binding, macrophage colony stimulating factor receptor binding, macrophage colony-stimulating factor receptor ligand Relationships: is a type of cytokine receptor binding [GO:0005126]